2-alkenal reductase [NAD(P)H] activity [GO:0032440] (molecular function) References: PMID:16299173 Sources: EC:1.3.1.74 Subtypes: GO:0035798 Relationships: is a type of oxidoreductase activity, acting on the CH-CH group of donors, NAD or NADP as acceptor [GO:0016628] Also known as: 2-alkenal reductase [NAD(P)+] activity, NAD(P)H-dependent alkenal/one oxidoreductase activity, n-alkanal:NAD(P)+ 2-oxidoreductase activity Definition: Catalysis of the reaction: n-alkanal + NAD(P)+ = alk-2-enal + NAD(P)H + H+.